{
  "term_id": "GO:0004565",
  "gene_name": "Beta-galactosidase-1-like protein",
  "gene": "UniProtKB:Q6UWU2",
  "term_label": "beta-galactosidase activity",
  "gene_symbol": "GLB1L"
}